{
  "term_id": "UNKNOWN:0003",
  "gene_name": "Glycerol-3-phosphate acyltransferase 3",
  "gene": "UniProtKB:Q53EU6",
  "gene_symbol": "GPAT3",
  "term_label": "Unknown cellular component"
}